complement component C3a binding [GO:0001850] (molecular function) Definition: Binding to a C3a product of the complement cascade. Relationships: is a type of complement binding [GO:0001848] Sources: GOC:add, ISBN:0781735149